natural killer cell apoptotic process [GO:0070246] (BP) Relationships: is a type of GO:0070227 Regulation: regulated by regulation of natural killer cell apoptotic process [GO:0070247]; RO_0002212 by negative regulation of natural killer cell apoptotic process [GO:0070248]; positively regulated by positive regulation of natural killer cell apoptotic process [GO:0070249] References: PMID:15728472 Sources: CL:0000623, GOC:add, GOC:mtg_apoptosis Also known as: NK cell apoptosis, natural killer cell apoptosis Definition: Any apoptotic process in a natural killer cell, a lymphocyte that can spontaneously kill a variety of target cells without prior antigenic activation.